positive regulation of complement activation, alternative pathway [GO:0045958] (biological process) Definition: Any process that activates or increases the frequency, rate or extent of complement activation by the alternative pathway. Also known as: positive regulation of complement cascade, alternative pathway, up regulation of complement activation, alternative pathway, up-regulation of complement activation, alternative pathway, upregulation of complement activation, alternative pathway, activation of complement activation, alternative pathway, stimulation of complement activation, alternative pathway Sources: GOC:go_curators Relationships: is a type of regulation of complement activation, alternative pathway [GO:0030451]; is a type of positive regulation of innate immune response [GO:0045089]; is_a positive regulation of complement activation [GO:0045917]; positively regulates complement activation, alternative pathway [GO:0006957]